D-xylulokinase activity [GO:0004856] (molecular function) Also known as: xylulokinase activity, ATP:D-xylulose 5-phosphotransferase activity, xylulokinase (phosphorylating), xylulose kinase activity Sources: EC:2.7.1.17, RHEA:10964 Relationships: is a type of GO:0016773; is a type of carbohydrate kinase activity [GO:0019200] Definition: Catalysis of the reaction: D-xylulose + ATP = D-xylulose 5-phosphate + ADP + H+.